{
  "gene_symbol": "SAMD8",
  "term_id": "GO:0005789",
  "term_label": "endoplasmic reticulum membrane",
  "gene": "UniProtKB:Q96LT4",
  "gene_name": "Sphingomyelin synthase-related protein 1"
}